response to nematicide [GO:0093002] (biological process) Also known as: response to antihelmintic, response to nematocide Definition: Any process that results in a change in state or activity of a cell or an organism (in terms of movement, secretion, enzyme production, gene expression, etc.) as a result of a nematicide stimulus. Nematicides are chemicals used to kill nematodes. Relationships: is a type of response to toxic substance [GO:0009636] References: PMID:22301316 Sources: GOC:kvm